{
  "gene_name": "Putative zinc finger protein 876",
  "term_id": "UNKNOWN:0003",
  "gene_symbol": "ZNF876P",
  "gene": "UniProtKB:Q49A33",
  "term_label": "Unknown cellular component"
}